non-tyrosine kinase fibroblast growth factor receptor activity [GO:0001571] (molecular function) References: PMID:11418238 Sources: GOC:signaling Definition: Combining with fibroblast growth factor (FGF) and transmitting the signal from one side of the membrane to the other by a mechanism independent of tyrosine kinase activity. Also known as: non-tyrosine kinase FGF receptor activity, non-tyrosine kinase FGFR activity Relationships: is a type of transmembrane signaling receptor activity [GO:0004888]